{
  "gene_symbol": "SHE",
  "term_id": "GO:0001784",
  "gene_name": "SH2 domain-containing adapter protein E",
  "term_label": "phosphotyrosine residue binding",
  "gene": "UniProtKB:Q5VZ18"
}